{
  "term_label": "Unknown molecular function",
  "gene_name": "Bridge-like lipid transfer protein family member 2",
  "gene": "UniProtKB:Q14667",
  "gene_symbol": "BLTP2",
  "term_id": "UNKNOWN:0001"
}